{
  "term_label": "cell projection assembly",
  "gene_symbol": "RAC3",
  "term_id": "GO:0030031",
  "gene_name": "Ras-related C3 botulinum toxin substrate 3",
  "gene": "UniProtKB:P60763"
}